{
  "gene_name": "One cut domain family member 3",
  "gene": "UniProtKB:O60422",
  "term_id": "GO:0005634",
  "term_label": "nucleus",
  "gene_symbol": "ONECUT3"
}